response to hydrostatic pressure [GO:0051599] (biological process) Definition: Any process that results in a change in state or activity of a cell or an organism (in terms of movement, secretion, enzyme production, gene expression, etc.) as a result of a hydrostatic pressure stimulus. Hydrostatic pressure is the force acting on an object in a system where the fluid is at rest (as opposed to moving). The weight of the fluid above the object creates pressure on it. Relationships: is a type of response to stress [GO:0006950]; is a type of response to water [GO:0009415] Also known as: response to biomechanical stress, response to static fluid pressure Subtypes: cellular response to hydrostatic pressure [GO:0071464] Sources: Wikipedia:Hydrostatic_pressure